6-phosphofructokinase complex [GO:0005945] (CC) Definition: A protein complex that possesses 6-phosphofructokinase activity; homodimeric, homooctameric, and allosteric homotetrameric forms are known. Sources: GOC:mah, GOC:vw, ISBN:0198506732 Relationships: is a type of transferase complex, transferring phosphorus-containing groups [GO:0061695]; is part of cytosol [GO:0005829]